{
  "term_label": "nucleus",
  "term_id": "GO:0005634",
  "gene": "UniProtKB:Q92688",
  "gene_symbol": "ANP32B",
  "gene_name": "Acidic leucine-rich nuclear phosphoprotein 32 family member B"
}